hydrolase activity, acting on acid phosphorus-nitrogen bonds [GO:0016825] (molecular function) Sources: EC:3.9.1.- Definition: Catalysis of the hydrolysis of any acid phosphorus-nitrogen bond. Subtypes: GO:0050187, protein arginine phosphatase activity [GO:0098627], GO:0101006 Relationships: is a type of GO:0016787